nucleobase transmembrane transporter activity [GO:0015205] (MF) Sources: ISBN:0198506732 Subtypes: purine nucleobase transmembrane transporter activity [GO:0005345], pyrimidine nucleobase transmembrane transporter activity [GO:0005350], GO:0015391 Definition: Enables the transfer of a nucleobase, any nitrogenous base that is a constituent of a nucleoside, nucleotide, or nucleic acidfrom one side of a membrane to the other. Relationships: is a type of transmembrane transporter activity [GO:0022857]; is part of nucleobase transport [GO:0015851]